positive regulation of male germ cell proliferation [GO:2000256] (biological process) Relationships: is a type of GO:1905938; is a type of GO:2000243; is a type of GO:2000254; positively regulates GO:0002176 Sources: GOC:obol Definition: Any process that activates or increases the frequency, rate or extent of male germ cell proliferation.